positive regulation of eating behavior [GO:1904000] (biological process) References: PMID:11961051 Sources: GOC:TermGenie, GO_REF:0000058 Also known as: positive regulation of eating behaviour, up regulation of eating behavior, up regulation of eating behaviour, up-regulation of eating behavior, up-regulation of eating behaviour, upregulation of eating behavior, upregulation of eating behaviour, activation of eating behavior, activation of eating behaviour Definition: Any process that activates or increases the frequency, rate or extent of eating behavior. Relationships: is a type of regulation of eating behavior [GO:1903998]; is a type of positive regulation of feeding behavior [GO:2000253]; positively regulates GO:0042755 Subtypes: positive regulation of nematode pharyngeal pumping [GO:1903746]